{
  "term_label": "Unknown biological process",
  "gene": "UniProtKB:Q5U649",
  "gene_name": "Uncharacterized protein C12orf60",
  "gene_symbol": "C12orf60",
  "term_id": "UNKNOWN:0002"
}